{
  "term_label": "cytosol",
  "gene_symbol": "HSP90AB3P",
  "gene": "UniProtKB:Q58FF7",
  "gene_name": "Putative heat shock protein HSP 90-beta-3",
  "term_id": "GO:0005829"
}